{
  "term_id": "GO:0016581",
  "term_label": "NuRD complex",
  "gene_symbol": "MTA1",
  "gene_name": "Metastasis-associated protein MTA1",
  "gene": "UniProtKB:Q13330"
}